{
  "term_label": "cell surface receptor signaling pathway",
  "gene_name": "T cell receptor beta variable 7-2",
  "term_id": "GO:0007166",
  "gene": "UniProtKB:A0A1B0GXF2",
  "gene_symbol": "TRBV7-2"
}